linoleate 8R-lipoxygenase activity [GO:0052878] (molecular function) Definition: Catalysis of the reaction: O2 + linoleate = (8R,9Z,12Z)-8-hydroperoxyoctadeca-9,12-dienoate. Sources: RHEA:25395 Also known as: 5,8-LDS (bifunctional enzyme) activity, 5,8-linoleate diol synthase (bifunctional enzyme) activity, 7,8-LDS (bifunctional enzyme) activity, 7,8-linoleate diol synthase (bifunctional enzyme) activity, linoleate diol synthase activity Relationships: is a type of oxidoreductase activity, acting on single donors with incorporation of molecular oxygen, incorporation of two atoms of oxygen [GO:0016702]